modified histidine catabolic process [GO:0052702] (biological process) Definition: The chemical reactions and pathways resulting in the breakdown of compounds derived from histidine, 2-amino-3-(1H-imidazol-4-yl)propanoic acid. Sources: GOC:ai Also known as: cellular histidine derivative breakdown, cellular histidine derivative catabolic process, cellular histidine derivative catabolism, cellular histidine derivative degradation, cellular modified histidine breakdown, cellular modified histidine catabolic process, cellular modified histidine catabolism, cellular modified histidine degradation, histidine derivative catabolic process, modified histidine catabolism Relationships: is a type of modified amino acid catabolic process [GO:0042219] Subtypes: GO:0052700